{
  "term_label": "mechanosensitive monoatomic ion channel activity",
  "gene_symbol": "TMC1",
  "gene_name": "Transmembrane channel-like protein 1",
  "term_id": "GO:0008381",
  "gene": "UniProtKB:Q8TDI8"
}